{
  "term_label": "mitochondrial fatty acid beta-oxidation multienzyme complex",
  "gene": "UniProtKB:P40939",
  "gene_name": "Trifunctional enzyme subunit alpha, mitochondrial",
  "gene_symbol": "HADHA",
  "term_id": "GO:0016507"
}